{
  "gene_symbol": "GUCA1ANB",
  "term_id": "UNKNOWN:0001",
  "term_label": "Unknown molecular function",
  "gene": "UniProtKB:X6R8D5",
  "gene_name": "Putative uncharacterized protein GUCA1ANB"
}